regulation of establishment of Sertoli cell barrier [GO:1904444] (biological process) Also known as: regulation of establishment of BTB, regulation of establishment of SCB, regulation of establishment of blood-testis barrier References: PMID:18057314 Sources: GOC:TermGenie, GO_REF:0000058 Relationships: is a type of regulation of cell development [GO:0060284]; is a type of regulation of reproductive process [GO:2000241]; regulates establishment of Sertoli cell barrier [GO:0097368] Definition: Any process that modulates the frequency, rate or extent of establishment of Sertoli cell barrier. Subtypes: GO:1904445, GO:1904446